{
  "term_id": "GO:0031507",
  "term_label": "heterochromatin formation",
  "gene_symbol": "HDAC1",
  "gene_name": "Histone deacetylase 1",
  "gene": "UniProtKB:Q13547"
}